{
  "gene": "UniProtKB:Q9NXH3",
  "term_label": "Unknown cellular component",
  "gene_name": "Protein phosphatase 1 regulatory subunit 14D",
  "gene_symbol": "PPP1R14D",
  "term_id": "UNKNOWN:0003"
}